{
  "term_label": "extracellular region",
  "gene_name": "4-galactosyl-N-acetylglucosaminide 3-alpha-L-fucosyltransferase FUT6",
  "gene": "UniProtKB:P51993",
  "term_id": "GO:0005576",
  "gene_symbol": "FUT6"
}